mannose transmembrane transport [GO:0015761] (biological process) Relationships: is a type of GO:0008645 Definition: The process in which mannose is transported across a lipid bilayer, from one side of a membrane to the other. Mannose is the aldohexose manno-hexose, the C-2 epimer of glucose. The D-(+)-form is widely distributed in mannans and hemicelluloses and is of major importance in the core oligosaccharide of N-linked oligosaccharides of glycoproteins. Sources: GOC:ai Also known as: mannose transport